regulation of basidium development [GO:0075314] (biological process) Relationships: is a type of regulation of spore-bearing organ development [GO:0075260]; regulates GO:0075313 Sources: GOC:pamgo_curators Subtypes: positive regulation of basidium development [GO:0075315], negative regulation of basidium development [GO:0075316] Definition: Any process that modulates the frequency, rate or extent of basidium development, a process that leads to the formation of a basidium, a small, specialized club-shaped structure typically bearing four basidiospores at the tips of minute projections. The basidium is unique to Basidiomycetes and distinguishes them from other kinds of fungi.